{
  "gene_symbol": "PIK3R4",
  "term_id": "GO:0034271",
  "gene": "UniProtKB:Q99570",
  "term_label": "phosphatidylinositol 3-kinase complex, class III, type I",
  "gene_name": "Phosphoinositide 3-kinase regulatory subunit 4"
}